dauer larval development [GO:0040024] (biological process) Regulation: RO_0002211 by GO:0061065; positively regulated by positive regulation of dauer larval development [GO:0061066]; negatively regulated by negative regulation of dauer larval development [GO:0061067] Relationships: is a type of nematode larval development [GO:0002119] Definition: The process whose specific outcome is the progression of the dauer larva over time, through the facultative diapause of the dauer (enduring) larval stage, with specialized traits adapted for dispersal and long-term survival, with elevated stress resistance and without feeding. Sources: GOC:ems, ISBN:087969307X